calmodulin-activated 3',5'-cyclic-GMP phosphodiesterase activity [GO:0048101] (MF) Definition: Catalysis of the reactions: nucleoside 3',5'-cyclic GMP + H2O = GMP + H+; this activity is activated by binding to calcium-bound calmodulin. Relationships: is a type of 3',5'-cyclic-GMP phosphodiesterase activity [GO:0047555] Also known as: calcium- and calmodulin-regulated 3',5'-cyclic-GMP phosphodiesterase activity, calcium- and calmodulin-regulated cGMP-specific phosphodiesterase activity, calcium- and calmodulin-regulated cyclic-GMP phosphodiesterase activity, calcium/calmodulin-regulated cGMP-specific phosphodiesterase activity, calcium- and calmodulin-regulated cGMP phosphodiesterase activity References: PMID:35216259 Sources: GOC:jid